endoplasmic reticulum subcompartment [GO:0098827] (CC) Subtypes: GO:0014802, GO:0016029, GO:0071781, endoplasmic reticulum tubular network [GO:0071782] Relationships: is a type of GO:0031984; is part of GO:0005783 Sources: GOC:dos Definition: A distinct region of the endoplasmic reticulum.